S-shaped body morphogenesis [GO:0072050] (biological process) Relationships: is a type of anatomical structure morphogenesis [GO:0009653]; is part of nephron morphogenesis [GO:0072028] Subtypes: mesonephric S-shaped body morphogenesis [GO:0061244], metanephric S-shaped body morphogenesis [GO:0072284] Definition: The process in which the S-shaped body is generated and organized. The S-shaped body is the successor of the comma-shaped body that contributes to the morphogenesis of the nephron. Sources: GOC:mtg_kidney_jan10